response to 4'-epidoxorubicin [GO:1902522] (biological process) Also known as: response to epirubicin Definition: Any process that results in a change in state or activity of a cell or an organism (in terms of movement, secretion, enzyme production, gene expression, etc.) as a result of a 4'-epidoxorubicin stimulus. Note: Note that this term is in the subset of terms that should not be used for direct manual annotation of gene products. It was created to be used for cross-referencing by other ontologies. Direct annotations to this term may be amended during annotation QC. Relationships: is_a response to alcohol [GO:0097305]; is a type of response to ketone [GO:1901654]; is a type of GO:1901698; is a type of response to glycoside [GO:1903416] References: PMID:23648065 Sources: GOC:TermGenie, GOC:dw